cellular response to alkyl hydroperoxide [GO:0071448] (biological process) Sources: GOC:mah Definition: Any process that results in a change in state or activity of a cell (in terms of movement, secretion, enzyme production, gene expression, etc.) as a result of an alkyl hydroperoxide stimulus. Alkyl hydroperoxides are monosubstitution products of hydrogen peroxide, HOOH, where the substituent is an alkyl group. Subtypes: cellular response to tert-butyl hydroperoxide [GO:0072736] Relationships: is a type of response to alkyl hydroperoxide [GO:0033195]; is_a cellular response to hydroperoxide [GO:0071447]